xylono-1,4-lactonase activity [GO:0050402] (molecular function) Also known as: D-xylono-1,4-lactone lactonohydrolase activity, xylono-g-lactonase activity, xylonolactonase activity Relationships: is a type of GO:0052689 Sources: EC:3.1.1.68 Definition: Catalysis of the reaction: D-xylono-1,4-lactone + H2O = D-xylonate.